{
  "gene": "UniProtKB:P48444",
  "term_id": "GO:0051645",
  "gene_name": "Coatomer subunit delta",
  "gene_symbol": "ARCN1",
  "term_label": "Golgi localization"
}